{
  "term_label": "neuron projection development",
  "term_id": "GO:0031175",
  "gene_symbol": "STMN1",
  "gene_name": "Stathmin",
  "gene": "UniProtKB:P16949"
}